{
  "term_id": "GO:0030239",
  "gene_symbol": "LMOD1",
  "gene": "UniProtKB:P29536",
  "gene_name": "Leiomodin-1",
  "term_label": "myofibril assembly"
}